retromer complex [GO:0030904] (cellular component) Definition: A conserved hetero-pentameric membrane-associated complex involved in retrograde transport from endosomes to the Golgi apparatus. The budding yeast retromer comprises Vps35p, Vps29p, Vps26p, Vps5p, and Vps17p. The mammalian complex shows slight variation in composition compared to yeast, and comprises SNX1 or SNX2, SNX5 or SNX6, VPS26A or VPS26B, VPS29, and VPS35. Relationships: is a type of membrane protein complex [GO:0098796]; is part of endomembrane system [GO:0012505] References: PMID:26220253, PMID:27385586, PMID:9700157 Sources: GOC:bf